{
  "gene_symbol": "SMC5",
  "gene_name": "Structural maintenance of chromosomes protein 5",
  "term_label": "nucleus",
  "term_id": "GO:0005634",
  "gene": "UniProtKB:Q8IY18"
}